{
  "term_label": "cytoplasm",
  "term_id": "GO:0005737",
  "gene_symbol": "TGFBRAP1",
  "gene_name": "Transforming growth factor-beta receptor-associated protein 1",
  "gene": "UniProtKB:Q8WUH2"
}